{
  "term_id": "GO:0060213",
  "gene": "UniProtKB:P62487",
  "gene_symbol": "POLR2G",
  "gene_name": "DNA-directed RNA polymerase II subunit RPB7",
  "term_label": "positive regulation of nuclear-transcribed mRNA poly(A) tail shortening"
}